dihydroorotate dehydrogenase (NAD+) activity [GO:0004589] (molecular function) Definition: Catalysis of the reaction: (S)-dihydroorotate + NAD+ = H+ + NADH + orotate. Sources: RHEA:13513 Also known as: orotate reductase (NADH) activity, (S)-dihydroorotate:NAD+ oxidoreductase activity Relationships: is_a dihydroorotate dehydrogenase activity [GO:0004152]; is a type of oxidoreductase activity, acting on the CH-CH group of donors, NAD or NADP as acceptor [GO:0016628]